A band [GO:0031672] (cellular component) Also known as: A disc, Q disc, anisotropic disc, transverse disc Definition: The dark-staining region of a sarcomere, in which myosin thick filaments are present; the center is traversed by the paler H zone, which in turn contains the M line. Sources: ISBN:0321204131 Relationships: is a type of cellular anatomical structure [GO:0110165]; is part of GO:0030017